negative regulation of HRI-mediated signaling [GO:0141191] (biological process) Relationships: is_a GO:0065007 References: PMID:38297121 Definition: Any process that stops, prevents, or reduces the frequency, rate or extent of HRI-mediated signaling.